regulation of tRNA catabolic process [GO:1902370] (biological process) Also known as: regulation of tRNA breakdown, regulation of tRNA catabolism, regulation of tRNA degradation Subtypes: regulation of tRNA stability [GO:0036415], GO:1902371, positive regulation of tRNA catabolic process [GO:1902372] Relationships: is a type of regulation of catabolic process [GO:0009894]; is a type of regulation of tRNA metabolic process [GO:1903326]; regulates tRNA decay [GO:0016078] Sources: GOC:TermGenie, GOC:bf Definition: Any process that modulates the frequency, rate or extent of tRNA catabolic process.